{
  "gene_name": "Olfactory receptor 11G2",
  "gene_symbol": "OR11G2",
  "term_id": "UNKNOWN:0003",
  "term_label": "Unknown cellular component",
  "gene": "UniProtKB:Q8NGC1"
}